pilus shaft [GO:0009418] (cellular component) Definition: The long, slender, mid section of a pilus. Also known as: fimbrial shaft Sources: GOC:jl Relationships: is a type of cellular anatomical structure [GO:0110165]; is part of pilus [GO:0009289]